protein O-acetylglucosaminyltransferase activity [GO:0097363] (molecular function) Subtypes: RNA polymerase II C-terminal domain O-GlcNAc transferase activity [GO:0140841] Definition: Catalysis of the reaction: UDP-N-acetyl-D-glucosamine + [protein]-L-serine = UDP + [protein]-3-O-(N-acetyl-D-glucosaminyl)-L-serine, or UDP-N-acetyl-D-glucosamine + [protein]-L-threonine = UDP + [protein]-3-O-(N-acetyl-D-glucosaminyl)-L-threonine. References: PMID:22158438 Sources: GOC:jsg, GOC:sart Also known as: O-GlcNAc transferase, O-linked N-acetylglucosaminyltransferase, OGTase, UDP-N-acetyl-D-glucosamine:protein-O-beta-N-acetyl-D-glucosaminyl transferase, protein O-GlcNAc transferase activity Relationships: is a type of acetylglucosaminyltransferase activity [GO:0008375]; is a type of GO:0140096